{
  "term_id": "GO:0002286",
  "gene_name": "Interferon alpha-8",
  "gene": "UniProtKB:P32881",
  "gene_symbol": "IFNA8",
  "term_label": "T cell activation involved in immune response"
}